{
  "term_label": "adenosine 5'-(hexahydrogen pentaphosphate) catabolic process",
  "gene": "UniProtKB:Q8NFP7",
  "gene_symbol": "NUDT10",
  "term_id": "GO:1901911",
  "gene_name": "Diphosphoinositol polyphosphate phosphohydrolase 3-alpha"
}